{
  "gene_name": "U8 snoRNA-decapping enzyme",
  "term_label": "nucleus",
  "term_id": "GO:0005634",
  "gene": "UniProtKB:Q96DE0",
  "gene_symbol": "NUDT16"
}